{
  "term_label": "protein import into mitochondrial matrix",
  "term_id": "GO:0030150",
  "gene_name": "Mitochondrial import receptor subunit TOM40B",
  "gene": "UniProtKB:Q969M1",
  "gene_symbol": "TOMM40L"
}